{
  "gene_symbol": "GGTLC3",
  "term_id": "UNKNOWN:0002",
  "gene": "UniProtKB:B5MD39",
  "term_label": "Unknown biological process",
  "gene_name": "Putative glutathione hydrolase light chain 3"
}